sodium ion binding [GO:0031402] (molecular function) Sources: GOC:mah Relationships: is a type of alkali metal ion binding [GO:0031420] Also known as: Na+ ion binding Definition: Binding to a sodium ion (Na+).